regulation of interleukin-1-mediated signaling pathway [GO:2000659] (biological process) Definition: Any process that modulates the frequency, rate or extent of interleukin-1-mediated signaling pathway. Subtypes: negative regulation of interleukin-1-mediated signaling pathway [GO:2000660], GO:2000661 Relationships: is a type of GO:0001959; regulates interleukin-1-mediated signaling pathway [GO:0070498] Sources: GOC:obol Also known as: regulation of IL-1-mediated signaling pathway, regulation of interleukin-1-mediated signalling pathway, regulation of IL-1 alpha-mediated signaling pathway, regulation of IL-1 beta-mediated signaling pathway, regulation of interleukin-1 alpha-mediated signaling pathway, regulation of interleukin-1 beta-mediated signaling pathway